{
  "gene": "UniProtKB:P57087",
  "gene_name": "Junctional adhesion molecule B",
  "gene_symbol": "JAM2",
  "term_id": "GO:0070160",
  "term_label": "tight junction"
}